positive regulation of Ras protein signal transduction [GO:0046579] (biological process) Also known as: up regulation of Ras protein signal transduction, up-regulation of Ras protein signal transduction, upregulation of Ras protein signal transduction, activation of Ras protein signal transduction, stimulation of Ras protein signal transduction Relationships: is_a GO:0046578; is a type of GO:0051057; positively regulates GO:0007265 Sources: GOC:bf Definition: Any process that activates or increases the frequency, rate or extent of Ras protein signal transduction.